{
  "gene_name": "Ankyrin repeat and SOCS box protein 18",
  "term_label": "Unknown cellular component",
  "gene": "UniProtKB:Q6ZVZ8",
  "term_id": "UNKNOWN:0003",
  "gene_symbol": "ASB18"
}